{
  "gene": "UniProtKB:Q5SSJ5",
  "gene_symbol": "HP1BP3",
  "term_id": "GO:0031491",
  "term_label": "nucleosome binding",
  "gene_name": "Heterochromatin protein 1-binding protein 3"
}